{
  "gene_symbol": "NEIL1",
  "gene_name": "Endonuclease 8-like 1",
  "term_id": "GO:0005634",
  "term_label": "nucleus",
  "gene": "UniProtKB:Q96FI4"
}